{
  "gene_symbol": "JCAD",
  "term_id": "GO:0032587",
  "term_label": "ruffle membrane",
  "gene_name": "Junctional cadherin 5-associated protein",
  "gene": "UniProtKB:Q9P266"
}